{
  "gene_name": "Helicase SRCAP",
  "gene_symbol": "SRCAP",
  "gene": "UniProtKB:Q6ZRS2",
  "term_id": "GO:0000812",
  "term_label": "Swr1 complex"
}